{
  "term_id": "GO:0000785",
  "gene_name": "Transcription factor 7-like 1",
  "gene_symbol": "TCF7L1",
  "gene": "UniProtKB:Q9HCS4",
  "term_label": "chromatin"
}